{
  "gene_symbol": "BRD8",
  "gene_name": "Bromodomain-containing protein 8",
  "term_label": "Unknown biological process",
  "gene": "UniProtKB:Q9H0E9",
  "term_id": "UNKNOWN:0002"
}